{
  "term_label": "L-cystine transport",
  "gene_symbol": "CTNS",
  "gene": "UniProtKB:O60931",
  "gene_name": "Cystinosin",
  "term_id": "GO:0015811"
}